{
  "gene": "UniProtKB:Q86SJ2",
  "gene_name": "Amphoterin-induced protein 2",
  "term_id": "GO:0007420",
  "term_label": "brain development",
  "gene_symbol": "AMIGO2"
}